{
  "term_label": "antibacterial humoral response",
  "gene_name": "Ribonuclease K6",
  "term_id": "GO:0019731",
  "gene_symbol": "RNASE6",
  "gene": "UniProtKB:Q93091"
}